{
  "gene_symbol": "POGK",
  "gene": "UniProtKB:Q9P215",
  "term_label": "DNA binding",
  "term_id": "GO:0003677",
  "gene_name": "Pogo transposable element with KRAB domain"
}